{
  "gene_symbol": "IHH",
  "gene": "UniProtKB:Q14623",
  "gene_name": "Indian hedgehog protein",
  "term_label": "regulation of gene expression",
  "term_id": "GO:0010468"
}